{
  "gene_symbol": "SLC26A5",
  "term_label": "sulfate transmembrane transporter activity",
  "gene": "UniProtKB:P58743",
  "gene_name": "Prestin",
  "term_id": "GO:0015116"
}